Shc-Grb2-Sos complex [GO:0070619] (cellular component) Also known as: Shc-Grb2-mSos1 complex, EGF stimulated References: PMID:7970708, PMID:8940013 Sources: GOC:mah Definition: A protein complex that contains Grb2, the adaptor protein Shc and the guanine nucleotide exchange factor Sos (or an ortholog thereof, such as mSos1), and is involved in linking EGFR activation to the p21-Ras pathway. Relationships: is a type of plasma membrane protein complex [GO:0098797]